skeletal muscle atrophy [GO:0014732] (biological process) Definition: A process, occurring in skeletal muscle, that is characterized by a decrease in protein content, fiber diameter, force production and fatigue resistance in response to different conditions such as starvation, aging and disuse. Relationships: is a type of GO:0014891; is a type of GO:0043501 Sources: GOC:mtg_muscle